{
  "term_id": "UNKNOWN:0001",
  "gene": "UniProtKB:A5D6W6",
  "gene_symbol": "FITM1",
  "term_label": "Unknown molecular function",
  "gene_name": "Fat storage-inducing transmembrane protein 1"
}